glycogen phosphorylase activity [GO:0008184] (molecular function) Definition: Catalysis of the reaction: glycogen + phosphate = maltodextrin + alpha-D-glucose 1-phosphate. Sources: MetaCyc:GLYCOPHOSPHORYL-RXN Relationships: is a type of 1,4-alpha-oligoglucan phosphorylase activity [GO:0004645]